{
  "gene_symbol": "KCNC4",
  "gene_name": "Potassium voltage-gated channel subfamily C member 4",
  "term_id": "GO:0071805",
  "gene": "UniProtKB:Q03721",
  "term_label": "potassium ion transmembrane transport"
}